{
  "gene": "UniProtKB:O60566",
  "gene_symbol": "BUB1B",
  "term_label": "mitotic spindle assembly checkpoint signaling",
  "gene_name": "Mitotic checkpoint serine_threonine-protein kinase BUB1 beta",
  "term_id": "GO:0007094"
}